{
  "gene": "UniProtKB:Q2NL67",
  "gene_symbol": "PARP6",
  "term_label": "endoplasmic reticulum tubular network",
  "term_id": "GO:0071782",
  "gene_name": "Protein mono-ADP-ribosyltransferase PARP6"
}